{
  "term_id": "GO:0005802",
  "gene_symbol": "CCDC186",
  "term_label": "trans-Golgi network",
  "gene": "UniProtKB:Q7Z3E2",
  "gene_name": "Coiled-coil domain-containing protein 186"
}